{
  "gene_symbol": "IL27",
  "term_label": "regulation of T-helper 1 cell differentiation",
  "term_id": "GO:0045625",
  "gene": "UniProtKB:Q8NEV9",
  "gene_name": "Interleukin-27 subunit alpha"
}